negative regulation of formation of translation preinitiation complex [GO:1901194] (biological process) Relationships: is a type of negative regulation of protein-containing complex assembly [GO:0031333]; is_a regulation of formation of translation preinitiation complex [GO:1901193]; is a type of negative regulation of cytoplasmic translational initiation [GO:1904689]; negatively regulates GO:0001731 Definition: Any process that stops, prevents or reduces the frequency, rate or extent of formation of translation preinitiation complex. Also known as: down regulation of formation of translation pre-initiation complex, down regulation of formation of translation preinitiation complex, down regulation of translation preinitiation complex assembly, down-regulation of formation of translation pre-initiation complex, down-regulation of formation of translation preinitiation complex, down-regulation of translation preinitiation complex assembly, downregulation of formation of translation pre-initiation complex, downregulation of formation of translation preinitiation complex, downregulation of translation preinitiation complex assembly, inhibition of formation of translation pre-initiation complex, inhibition of translation preinitiation complex assembly, negative regulation of formation of translation pre-initiation complex, negative regulation of translation preinitiation complex assembly, inhibition of formation of translation preinitiation complex Sources: GOC:TermGenie